high-affinity D-glucose:proton symporter activity [GO:0005358] (molecular function) Also known as: high-affinity hydrogen/glucose transporter activity, high-affinity hydrogen:glucose transporter activity, high-affinity glucose:proton symporter activity, high-affinity hydrogen:glucose symporter activity Sources: GOC:mtg_transport Relationships: is a type of D-glucose:proton symporter activity [GO:0005356] Definition: Enables the transfer of a solute or solutes from one side of a membrane to the other according to the reaction: glucose + H+ = glucose + H+. This activity is constitutive and therefore always present, regardless of demand. Symporter activity enables the active transport of a solute across a membrane by a mechanism whereby two or more species are transported together in the same direction in a tightly coupled process not directly linked to a form of energy other than chemiosmotic energy. In high-affinity transport the transporter is able to bind the solute even if it is only present at very low concentrations.